4-hydroxy-4-methyl-2-oxoglutarate aldolase activity [GO:0047443] (molecular function) Sources: EC:4.1.3.17 Also known as: 4-hydroxy-4-methyl-2-ketoglutarate aldolase activity, 4-hydroxy-4-methyl-2-oxoglutarate pyruvate-lyase (pyruvate-forming), 4-hydroxy-4-methyl-2-oxoglutarate pyruvate-lyase activity, gamma-methyl-gamma-hydroxy-alpha-ketoglutaric aldolase activity, pyruvate aldolase activity Definition: Catalysis of the reactions: 4-hydroxy-4-methyl-2-oxoglutarate = 2 pyruvate, and 2-hydroxy-4-oxobutane-1,2,4-tricarboxylate = oxaloacetate + pyruvate. Relationships: is a type of oxo-acid-lyase activity [GO:0016833]